{
  "gene_name": "Megakaryocyte and platelet inhibitory receptor G6b",
  "term_id": "UNKNOWN:0001",
  "gene": "UniProtKB:O95866",
  "gene_symbol": "MPIG6B",
  "term_label": "Unknown molecular function"
}